{
  "gene": "UniProtKB:Q13588",
  "gene_symbol": "GRAP",
  "term_id": "GO:0005154",
  "gene_name": "GRB2-related adapter protein",
  "term_label": "epidermal growth factor receptor binding"
}